{
  "gene_name": "E3 ubiquitin-protein ligase RNF38",
  "gene": "UniProtKB:Q9H0F5",
  "term_id": "UNKNOWN:0003",
  "gene_symbol": "RNF38",
  "term_label": "Unknown cellular component"
}